{
  "gene_symbol": "NPPA",
  "term_label": "receptor guanylyl cyclase signaling pathway",
  "term_id": "GO:0007168",
  "gene": "UniProtKB:P01160",
  "gene_name": "Natriuretic peptides A"
}